{
  "term_label": "cytosolic ribosome",
  "gene_symbol": "RPS27A",
  "gene_name": "Ubiquitin-ribosomal protein eS31 fusion protein",
  "term_id": "GO:0022626",
  "gene": "UniProtKB:P62979"
}